{
  "gene": "UniProtKB:Q96KQ4",
  "term_id": "GO:0005634",
  "gene_name": "Apoptosis-stimulating of p53 protein 1",
  "gene_symbol": "PPP1R13B",
  "term_label": "nucleus"
}